D-tagatose 6-phosphate catabolic process [GO:2001059] (biological process) Definition: The chemical reactions and pathways resulting in the breakdown of a D-tagatose 6-phosphate. Also known as: D-tagatose 6-phosphate catabolism Sources: GOC:mengo_curators Relationships: is a type of phosphate-containing compound metabolic process [GO:0006796]; is a type of organophosphate catabolic process [GO:0046434]; is_a GO:1901136